neural tube patterning [GO:0021532] (biological process) Sources: GOC:cls, GOC:dgh, GOC:dph, GOC:jid, GO_REF:0000021 Relationships: is_a regionalization [GO:0003002]; is part of neural tube development [GO:0021915] Definition: The regionalization process that regulates the coordinated growth that establishes the non-random spatial arrangement of the neural tube.